{
  "term_label": "nuclear polyadenylation-dependent snRNA catabolic process",
  "gene_name": "Exosome component 10",
  "term_id": "GO:0071037",
  "gene": "UniProtKB:Q01780",
  "gene_symbol": "EXOSC10"
}